{
  "gene_symbol": "BORCS8",
  "term_id": "GO:0099078",
  "gene": "UniProtKB:Q96FH0",
  "term_label": "BORC complex",
  "gene_name": "BLOC-1-related complex subunit 8"
}